{
  "term_label": "Unknown molecular function",
  "term_id": "UNKNOWN:0001",
  "gene": "UniProtKB:A0A075B6Y2",
  "gene_name": "T cell receptor alpha joining 35 (non-functional) (Fragment)",
  "gene_symbol": "TRAJ35"
}